{
  "gene_symbol": "SLC12A8",
  "gene_name": "Solute carrier family 12 member 8",
  "term_label": "cell volume homeostasis",
  "term_id": "GO:0006884",
  "gene": "UniProtKB:A0AV02"
}